atrial septum secundum morphogenesis [GO:0003290] (biological process) Sources: GOC:mtg_heart Definition: The process in which anatomical structure of an atrial septum secundum is generated and organized. Relationships: is a type of atrial septum morphogenesis [GO:0060413]; is part of septum secundum development [GO:0003285]